{
  "gene_name": "PABIR family member 2",
  "term_id": "GO:0004865",
  "term_label": "protein serine/threonine phosphatase inhibitor activity",
  "gene_symbol": "PABIR2",
  "gene": "UniProtKB:Q7Z309"
}